{
  "gene": "UniProtKB:P04000",
  "gene_symbol": "OPN1LW",
  "gene_name": "Long-wave-sensitive opsin 1",
  "term_id": "GO:0007602",
  "term_label": "phototransduction"
}